{
  "term_id": "GO:0007605",
  "gene_symbol": "USH1G",
  "gene": "UniProtKB:Q495M9",
  "gene_name": "pre-mRNA splicing regulator USH1G",
  "term_label": "sensory perception of sound"
}